{
  "gene_name": "TGF-beta receptor type-1",
  "term_label": "cellular response to growth factor stimulus",
  "gene_symbol": "TGFBR1",
  "gene": "UniProtKB:P36897",
  "term_id": "GO:0071363"
}